{
  "term_label": "protein tyrosine phosphatase activity",
  "gene_symbol": "PTPN22",
  "gene_name": "Tyrosine-protein phosphatase non-receptor type 22",
  "term_id": "GO:0004725",
  "gene": "UniProtKB:Q9Y2R2"
}